{
  "gene_name": "Neutral amino acid uniporter 4",
  "gene_symbol": "SLC36A4",
  "gene": "UniProtKB:Q6YBV0",
  "term_label": "vacuolar membrane",
  "term_id": "GO:0005774"
}